{
  "gene_name": "Kelch domain-containing protein 1",
  "term_id": "UNKNOWN:0003",
  "term_label": "Unknown cellular component",
  "gene": "UniProtKB:Q8N7A1",
  "gene_symbol": "KLHDC1"
}